nicotinamide riboside metabolic process [GO:0046495] (biological process) Definition: The chemical reactions and pathways involving nicotinamide riboside, the product of the formation of a glycosidic bond between ribose and nicotinamide. Sources: ISBN:0198506732 Also known as: N-ribosylnicotinamide metabolic process, nicotinamide riboside metabolism Relationships: is a type of GO:0070637 Subtypes: GO:0006738, nicotinamide riboside biosynthetic process [GO:0071590]